ribose isomerase activity [GO:0050261] (molecular function) Definition: Catalysis of the reaction: aldehydo-D-ribose = D-ribulose. Sources: RHEA:20796 Also known as: D-ribose aldose-ketose-isomerase activity, D-ribose isomerase activity, D-ribose ketol-isomerase activity Relationships: is a type of intramolecular oxidoreductase activity, interconverting aldoses and ketoses [GO:0016861]